{
  "gene_symbol": "DEFB106A",
  "gene_name": "Beta-defensin 106",
  "term_id": "UNKNOWN:0003",
  "gene": "UniProtKB:Q8N104",
  "term_label": "Unknown cellular component"
}